RNA polymerase I general transcription initiation factor activity [GO:0001181] (molecular function) Definition: A general transcription initiation factor activity that contributes to transcription start site selection and transcription initiation of genes transcribed by RNA polymerase I. Factors required for RNA polymerase I transcription initiation include upstream activation factor (UAF), core factor (CF), TATA binding protein (TBP) and RRN3. In all species characterized, RNA polymerase I transcribes a large polycistronic transcript that is processed into several mature rRNAs (3 or 4 depending on the species), including the large subunit rRNA (28S in humans), the small subunit rRNA (18S in humans), as well as one or two additional smaller rRNAs (the 5.8S rRNA in humans). In most species, this large rRNA transcript is the sole product of RNA polymerase I. However there are rare exceptions, such as Trypanosoma brucei, where RNA polymerase I also transcribes certain mRNAs. Also known as: core RNA polymerase I binding transcription factor activity, transcription factor activity, core RNA polymerase I binding, RNA polymerase I transcription general initiation factor activity, general RNA polymerase I transcription factor activity References: PMID:11500378, PMID:17972917, PMID:25346433, PMID:28340337, PMID:28842442, PMID:31358304 Sources: GOC:txnOH-2018 Relationships: is a type of general transcription initiation factor activity [GO:0140223]; is part of transcription by RNA polymerase I [GO:0006360]